{
  "term_label": "cytosine C-5 DNA demethylase activity",
  "gene": "UniProtKB:Q6NS38",
  "gene_name": "DNA oxidative demethylase ALKBH2",
  "gene_symbol": "ALKBH2",
  "term_id": "GO:0051747"
}